eye field cell fate commitment involved in camera-type eye formation [GO:0060898] (biological process) Sources: GOC:dph, GOC:sdb_2009, GOC:tb Definition: The commitment of neurectodermal cells to cells of the eye field and their capacity to differentiate into eye field cells. Eye field cells are neurectodermal cells that will form the optic placode. Relationships: is a type of cell fate commitment involved in pattern specification [GO:0060581]; BFO_0000050 lens placode formation involved in camera-type eye formation [GO:0046619]; is part of GO:0060897